{
  "term_label": "Unknown biological process",
  "gene_symbol": "NDUFB4",
  "gene_name": "NADH dehydrogenase [ubiquinone] 1 beta subcomplex subunit 4",
  "gene": "UniProtKB:O95168",
  "term_id": "UNKNOWN:0002"
}